plastid fission [GO:0043572] (biological process) Definition: The creation of two or more plastids by division of one plastid. A plastid is any member of a family of organelles found in the cytoplasm of plants and some protists, which are membrane-bounded and contain DNA. Subtypes: chloroplast fission [GO:0010020], GO:0043573 Relationships: is a type of organelle fission [GO:0048285] Sources: GOC:jl